{
  "gene_name": "Tripartite motif-containing protein 74",
  "term_label": "innate immune response",
  "gene": "UniProtKB:Q86UV6",
  "term_id": "GO:0045087",
  "gene_symbol": "TRIM74"
}